{
  "term_label": "mitochondrion",
  "gene_name": "Thymidylate synthase",
  "gene_symbol": "TYMS",
  "term_id": "GO:0005739",
  "gene": "UniProtKB:P04818"
}